{
  "gene": "UniProtKB:A0A1B0GUA6",
  "term_id": "UNKNOWN:0001",
  "gene_name": "Putative coiled-coil domain-containing protein 195",
  "term_label": "Unknown molecular function",
  "gene_symbol": "CCDC195"
}